{
  "gene_name": "Acid-sensing ion channel 1",
  "term_id": "GO:0098978",
  "gene": "UniProtKB:P78348",
  "term_label": "glutamatergic synapse",
  "gene_symbol": "ASIC1"
}